{
  "gene": "UniProtKB:Q9UQM7",
  "gene_symbol": "CAMK2A",
  "gene_name": "Calcium_calmodulin-dependent protein kinase type II subunit alpha",
  "term_id": "GO:0043005",
  "term_label": "neuron projection"
}